{
  "term_id": "UNKNOWN:0001",
  "term_label": "Unknown molecular function",
  "gene": "UniProtKB:A0A0A0MS06",
  "gene_name": "Probable non-functional T cell receptor beta variable 23-1",
  "gene_symbol": "TRBV23-1"
}